{
  "gene_name": "Mediator of RNA polymerase II transcription subunit 24",
  "term_label": "mediator complex",
  "gene_symbol": "MED24",
  "gene": "UniProtKB:O75448",
  "term_id": "GO:0016592"
}